{
  "term_id": "GO:0016324",
  "gene_symbol": "SLC34A2",
  "term_label": "apical plasma membrane",
  "gene": "UniProtKB:O95436",
  "gene_name": "Sodium-dependent phosphate transport protein 2B"
}